{
  "gene_name": "Sulfate anion transporter 1",
  "gene_symbol": "SLC26A1",
  "term_id": "GO:0005886",
  "gene": "UniProtKB:Q9H2B4",
  "term_label": "plasma membrane"
}